{
  "gene_name": "N(4)-(beta-N-acetylglucosaminyl)-L-asparaginase",
  "gene": "UniProtKB:P20933",
  "term_label": "N4-(beta-N-acetylglucosaminyl)-L-asparaginase activity",
  "term_id": "GO:0003948",
  "gene_symbol": "AGA"
}